{
  "gene_name": "Ribonuclease 7",
  "gene_symbol": "RNASE7",
  "term_label": "extracellular space",
  "gene": "UniProtKB:Q9H1E1",
  "term_id": "GO:0005615"
}